{
  "gene_symbol": "NELL1",
  "term_id": "GO:0005615",
  "gene_name": "Protein kinase C-binding protein NELL1",
  "gene": "UniProtKB:Q92832",
  "term_label": "extracellular space"
}